{
  "gene_symbol": "ZNF547",
  "gene_name": "Zinc finger protein 547",
  "term_label": "RNA polymerase II cis-regulatory region sequence-specific DNA binding",
  "term_id": "GO:0000978",
  "gene": "UniProtKB:Q8IVP9"
}